tetrapyrrole metabolic process [GO:0033013] (biological process) Sources: GOC:mah Regulation: regulated by regulation of tetrapyrrole metabolic process [GO:1901401] Relationships: is a type of metabolic process [GO:0008152] Subtypes: porphyrin-containing compound metabolic process [GO:0006778], cobalamin metabolic process [GO:0009235], tetrapyrrole biosynthetic process [GO:0033014], tetrapyrrole catabolic process [GO:0033015] Also known as: tetrapyrrole metabolism Definition: The chemical reactions and pathways involving tetrapyrroles, natural pigments containing four pyrrole rings joined by one-carbon units linking position 2 of one pyrrole ring to position 5 of the next.